double-strand break repair via alternative nonhomologous end joining [GO:0097681] (biological process) References: PMID:18584027, PMID:21655080 Sources: GOC:rph, Wikipedia:Microhomology-mediated_end_joining Relationships: is a type of double-strand break repair via nonhomologous end joining [GO:0006303] Definition: An instance of double-strand break repair via nonhomologous end joining that is independent of factors important for V(D)J recombination (as opposed to classical nonhomologous end joining). It often results in a deletion with microhomology (i.e. 5-25bp homology) at the repair junction. Among different subclasses of nonhomologous end joining (NHEJ), alternative NHEJ appears to play a significant role in the etiology of mutations that arise during cancer development and treatment. Also known as: double-strand break repair via microhomology-mediated end joining, A-NHEJ, MMEJ, alt-NHEJ